peptidase activator activity [GO:0016504] (molecular function) Sources: GOC:ai Relationships: is a type of enzyme activator activity [GO:0008047]; is a type of peptidase regulator activity [GO:0061134]; positively regulates peptidase activity [GO:0008233] Also known as: protease activator activity Definition: Binds to and increases the activity of a peptidase. Subtypes: peptidase activator activity involved in apoptotic process [GO:0016505], deubiquitinase activator activity [GO:0035800], GO:0061133